apolipoprotein B mRNA editing enzyme complex [GO:0030895] (cellular component) Definition: Protein complex that mediates editing of the mRNA encoding apolipoprotein B; catalyzes the deamination of C to U (residue 6666 in the human mRNA). Contains a catalytic subunit, APOBEC-1, and other proteins (e.g. human ASP; rat ASP and KSRP). Note: ASP = APOBEC1 complementation factor 1, a1cf, acf; KSRP = Khsrp (KH-type splicing regulatory protein) Also known as: APOBEC, apoB mRNA editing enzyme complex References: PMID:10781591, PMID:12683974 Relationships: is a type of GO:0045293; is_a nuclear protein-containing complex [GO:0140513]